{
  "gene_symbol": "POLA1",
  "term_id": "GO:0006273",
  "gene": "UniProtKB:P09884",
  "term_label": "lagging strand elongation",
  "gene_name": "DNA polymerase alpha catalytic subunit"
}